{
  "gene_name": "Neuronal acetylcholine receptor subunit alpha-2",
  "gene_symbol": "CHRNA2",
  "term_label": "acetylcholine-gated channel complex",
  "term_id": "GO:0005892",
  "gene": "UniProtKB:Q15822"
}